{
  "term_label": "cytoplasm",
  "term_id": "GO:0005737",
  "gene_name": "Rab-interacting lysosomal protein",
  "gene_symbol": "RILP",
  "gene": "UniProtKB:Q96NA2"
}